{
  "gene_name": "Zinc finger protein 280B",
  "term_id": "GO:0000978",
  "term_label": "RNA polymerase II cis-regulatory region sequence-specific DNA binding",
  "gene": "UniProtKB:Q86YH2",
  "gene_symbol": "ZNF280B"
}